3-(3-hydroxy)phenylpropionate catabolic process [GO:0019622] (biological process) Definition: The chemical reactions and pathways resulting in the breakdown of 3-(3-hydroxy)phenylpropionate, a hydroxylated derivative of phenylpropionate. Sources: GOC:ai Relationships: is a type of alcohol catabolic process [GO:0046164]; is a type of monocarboxylic acid catabolic process [GO:0072329] Also known as: 3-(3-hydroxy)phenylpropionate breakdown, 3-(3-hydroxy)phenylpropionate catabolism, 3-(3-hydroxy)phenylpropionate degradation